{
  "gene_symbol": "VPS26B",
  "term_id": "UNKNOWN:0001",
  "gene_name": "Vacuolar protein sorting-associated protein 26B",
  "gene": "UniProtKB:Q4G0F5",
  "term_label": "Unknown molecular function"
}